regulation of mediator complex assembly [GO:2001176] (biological process) Relationships: is a type of regulation of protein-containing complex assembly [GO:0043254]; regulates mediator complex assembly [GO:0036034] Definition: Any process that modulates the frequency, rate or extent of mediator complex assembly. Subtypes: negative regulation of mediator complex assembly [GO:2001177], positive regulation of mediator complex assembly [GO:2001178] Sources: GOC:obol